AMP-thymidine kinase activity [GO:0047667] (molecular function) Sources: EC:2.7.1.114, MetaCyc:AMP--THYMIDINE-KINASE-RXN Definition: Catalysis of the reaction: AMP + thymidine = adenosine + thymidine 5'-phosphate. Relationships: is a type of kinase activity [GO:0016301]; is_a phosphotransferase activity, alcohol group as acceptor [GO:0016773] Also known as: AMP:dThd kinase activity, AMP:deoxythymidine 5'-phosphotransferase activity, AMP:deoxythymidine kinase activity, AMP:thymidine 5'-phosphotransferase activity, adenylate-nucleoside phosphotransferase activity, adenylic acid:deoxythymidine 5'-phosphotransferase activity, thymidine phosphotransferase activity